hydroxymethylpyrimidine kinase activity [GO:0008902] (MF) Relationships: is a type of kinase activity [GO:0016301]; is a type of phosphotransferase activity, alcohol group as acceptor [GO:0016773] Definition: Catalysis of the reaction: 4-amino-5-hydroxymethyl-2-methylpyrimidine + ATP = 4-amino-2-methyl-5-phosphomethylpyrimidine + ADP + 2 H+. Also known as: ATP:4-amino-5-hydroxymethyl-2-methylpyrimidine 5-phosphotransferase activity, hydroxymethylpyrimidine kinase (phosphorylating) Sources: EC:2.7.1.49, RHEA:23096